{
  "gene_symbol": "DEFB128",
  "gene_name": "Beta-defensin 128",
  "term_label": "defense response to Gram-positive bacterium",
  "gene": "UniProtKB:Q7Z7B8",
  "term_id": "GO:0050830"
}